lamellipodium assembly [GO:0030032] (biological process) Sources: GOC:mah, ISBN:0815316194 Subtypes: GO:0003363 Also known as: lamellipodium biosynthesis, lamellipodium formation, lamellipodium biogenesis Relationships: is a type of lamellipodium organization [GO:0097581]; is a type of plasma membrane bounded cell projection assembly [GO:0120031] Definition: Formation of a lamellipodium, a thin sheetlike extension of the surface of a migrating cell. Regulation: regulated by GO:0010591; positively regulated by positive regulation of lamellipodium assembly [GO:0010592]; negatively regulated by negative regulation of lamellipodium assembly [GO:0010593]